{
  "term_id": "GO:0005886",
  "gene_symbol": "AMHR2",
  "term_label": "plasma membrane",
  "gene_name": "Anti-Muellerian hormone type-2 receptor",
  "gene": "UniProtKB:Q16671"
}